negative regulation of cell-glial cell adhesion involved in cerebral cortex lamination [GO:0021821] (biological process) Definition: The process that results in the release of migrating cells from their interaction with radial glial cells as a component of the process of cerebral cortex glial-mediated radial cell migration. References: PMID:12626695 Sources: GOC:cls, GOC:dgh, GOC:dph, GOC:jid, GO_REF:0000021 Relationships: is a type of GO:0022408; is part of layer formation in cerebral cortex [GO:0021819] Also known as: down regulation of cell-glial cell adhesion involved in cerebral cortex lamination, down-regulation of cell-glial cell adhesion involved in cerebral cortex lamination, downregulation of cell-glial cell adhesion involved in cerebral cortex lamination, inhibition of cell-glial cell adhesion involved in cerebral cortex lamination